phagocytic cup [GO:0001891] (cellular component) Definition: An invagination of the cell membrane formed by an actin dependent process during phagocytosis. Following internalization it is converted into a phagosome. References: PMID:10358769 Relationships: is_a cellular anatomical structure [GO:0110165]; is part of plasma membrane [GO:0005886]